response to iron(II) ion [GO:0010040] (biological process) Sources: GOC:sm Subtypes: cellular response to iron(II) ion [GO:0071282] Relationships: is a type of response to iron ion [GO:0010039] Also known as: response to iron(II) Definition: Any process that results in a change in state or activity of a cell or an organism (in terms of movement, secretion, enzyme production, gene expression, etc.) as a result of an iron(II) ion stimulus.